{
  "gene": "UniProtKB:Q9BSD3",
  "term_id": "GO:0000725",
  "gene_name": "RAD9, HUS1, RAD1-interacting nuclear orphan protein 1",
  "term_label": "recombinational repair",
  "gene_symbol": "RHNO1"
}